{
  "gene_name": "Chronic lymphocytic leukemia up-regulated protein 1",
  "term_label": "Unknown cellular component",
  "gene_symbol": "CLLU1",
  "gene": "UniProtKB:Q5K131",
  "term_id": "UNKNOWN:0003"
}